glutamate synthase (ferredoxin) activity [GO:0016041] (molecular function) Definition: Catalysis of the reaction: 2 L-glutamate + 2 oxidized ferredoxin = L-glutamine + 2-oxoglutarate + 2 reduced ferredoxin + 2 H+. This is a two-step reaction: (a) L-glutamate + NH3 = L-glutamine + H2O, (b) L-glutamate + 2 oxidized ferredoxin + H2O = NH3 + 2-oxoglutarate + 2 reduced ferredoxin + 2 H+. Sources: EC:1.4.7.1 Also known as: L-glutamate:ferredoxin oxidoreductase (transaminating), ferredoxin-dependent glutamate synthase activity, ferredoxin-glutamate synthase activity, glutamate synthase (ferredoxin-dependent) Note: Note that this term has a MetaCyc pathway reference as the pathway only has a single step. Relationships: is a type of glutamate synthase activity [GO:0015930]; is a type of oxidoreductase activity, acting on the CH-NH2 group of donors, iron-sulfur protein as acceptor [GO:0016643]